{
  "gene_name": "Olfactory receptor 1P1",
  "term_id": "GO:0007165",
  "term_label": "signal transduction",
  "gene": "UniProtKB:Q8NH06",
  "gene_symbol": "OR1P1"
}